{
  "gene_symbol": "SPTB",
  "term_id": "GO:0051015",
  "gene": "UniProtKB:P11277",
  "term_label": "actin filament binding",
  "gene_name": "Spectrin beta chain, erythrocytic"
}